{
  "gene": "UniProtKB:Q05048",
  "term_label": "Unknown molecular function",
  "gene_name": "Cleavage stimulation factor subunit 1",
  "gene_symbol": "CSTF1",
  "term_id": "UNKNOWN:0001"
}